alcohol transmembrane transporter activity [GO:0015665] (molecular function) Sources: ISBN:0198506732 Definition: Enables the transfer of an alcohol from one side of a membrane to the other. An alcohol is any carbon compound that contains a hydroxyl group. Relationships: is_a transmembrane transporter activity [GO:0022857] Subtypes: GO:0008493, cycloheximide transmembrane transporter activity [GO:0015243], fluconazole transmembrane transporter activity [GO:0015244], GO:0033288, GO:0034228, retinol transmembrane transporter activity [GO:0034632], GO:0042933, salicin transmembrane transporter activity [GO:0042950], glycolate transmembrane transporter activity [GO:0043879], GO:0051407, GO:0090440, GO:0097253, ABC-type doxorubicin transporter activity [GO:1901242]